1,4-alpha-glucan 6-alpha-glucosyltransferase activity [GO:0032001] (molecular function) Definition: Catalysis of the transfer an alpha-D-glucosyl residue in a (1->4)-alpha-D-glucan to the primary hydroxy group of glucose, free or combined in a (1->4)-alpha-D-glucan. Sources: EC:2.4.1.24 Relationships: is a type of glucosyltransferase activity [GO:0046527] Also known as: D-glucosyltransferase, 1,4-alpha-D-glucan 6-alpha-D-glucosyltransferase activity, 1,4-alpha-D-glucan:1,4-alpha-D-glucan(D-glucose) 6-alpha-D-glucosyltransferase activity, T-enzyme, oligoglucan-branching glycosyltransferase activity